protein targeting to chloroplast [GO:0045036] (biological process) Also known as: protein-chloroplast targeting Relationships: is a type of protein targeting [GO:0006605]; is a type of establishment of protein localization to chloroplast [GO:0072596] Sources: ISBN:0716731363 Definition: The process of directing proteins towards the chloroplast, usually using signals contained within the protein. Imported proteins are synthesized as cytosolic precursors containing N-terminal uptake-targeting sequences that direct each protein to its correct subcompartment and are subsequently cleaved.